{
  "term_label": "excitatory postsynaptic potential",
  "term_id": "GO:0060079",
  "gene_name": "Glutamate receptor ionotropic, NMDA 2D",
  "gene": "UniProtKB:O15399",
  "gene_symbol": "GRIN2D"
}